{
  "term_label": "peroxisomal membrane",
  "term_id": "GO:0005778",
  "gene_name": "Peroxisome biogenesis factor 2",
  "gene": "UniProtKB:P28328",
  "gene_symbol": "PEX2"
}